{
  "term_id": "GO:0004359",
  "gene_symbol": "NADSYN1",
  "gene": "UniProtKB:Q6IA69",
  "term_label": "glutaminase activity",
  "gene_name": "Glutamine-dependent NAD(+) synthetase"
}